{
  "gene": "UniProtKB:Q9NPA2",
  "gene_symbol": "MMP25",
  "gene_name": "Matrix metalloproteinase-25",
  "term_label": "extracellular matrix organization",
  "term_id": "GO:0030198"
}